cyclic 2,3-bisphospho-D-glycerate biosynthetic process [GO:1901369] (biological process) Definition: The chemical reactions and pathways resulting in the formation of cyclic 2,3-bisphospho-D-glyceric acid. Also known as: cDPG biosynthesis, cyclic 2,3-bisphospho-D-glyceric acid anabolism, cyclic 2,3-bisphospho-D-glyceric acid biosynthesis, cyclic 2,3-bisphospho-D-glyceric acid biosynthetic process, cyclic 2,3-bisphospho-D-glyceric acid formation, cyclic 2,3-bisphospho-D-glyceric acid synthesis, cyclic 2,3-diphosphoglycerate biosynthesis Relationships: is a type of phosphate-containing compound metabolic process [GO:0006796]; is a type of monocarboxylic acid biosynthetic process [GO:0072330]; is a type of organophosphate biosynthetic process [GO:0090407]; is a type of carbohydrate derivative biosynthetic process [GO:1901137] References: PMID:2226838 Sources: GOC:TermGenie, GOC:bf, GOC:crds